{
  "term_label": "structural constituent of ribosome",
  "gene_symbol": "RPS26P11",
  "gene": "UniProtKB:Q5JNZ5",
  "term_id": "GO:0003735",
  "gene_name": "Putative ribosomal protein eS26-like"
}